{
  "gene_name": "Frizzled-2",
  "gene_symbol": "FZD2",
  "term_id": "GO:0005886",
  "gene": "UniProtKB:Q14332",
  "term_label": "plasma membrane"
}